viral DNA genome replication [GO:0039693] (BP) Also known as: DNA-dependent viral DNA replication, viral DNA replication, viral DNA-dependent DNA replication Sources: GOC:bf, GOC:jl, VZ:915 Definition: The replication of a viral DNA genome. Relationships: is a type of GO:0019079; is a type of DNA biosynthetic process [GO:0071897] Subtypes: rolling hairpin viral DNA replication [GO:0039685], bidirectional double-stranded viral DNA replication [GO:0039686], viral DNA strand displacement replication [GO:0039687], viral double stranded DNA replication via reverse transcription [GO:0039688]